{
  "gene_symbol": "PHF1",
  "gene": "UniProtKB:O43189",
  "gene_name": "PHD finger protein 1",
  "term_label": "negative regulation of gene expression, epigenetic",
  "term_id": "GO:0045814"
}